pseudopodium organization [GO:0031268] (biological process) Definition: A process that is carried out at the cellular level which results in the assembly, arrangement of constituent parts, or disassembly of a pseudopodium, a temporary protrusion or retractile process of a cell, associated with cellular movement. Also known as: pseudopodium organisation, pseudopodium organization and biogenesis Sources: GOC:pg Subtypes: GO:0031269, pseudopodium retraction [GO:0031270] Relationships: is a type of plasma membrane bounded cell projection organization [GO:0120036]